cortical endoplasmic reticulum membrane [GO:0160219] (cellular component) Relationships: is a type of endoplasmic reticulum tubular network membrane [GO:0098826]; BFO_0000050 cortical endoplasmic reticulum [GO:0032541] References: PMID:32735772 Definition: The lipid bilayer surrounding the cortical endoplasmic reticulum.